{
  "term_label": "Unknown cellular component",
  "term_id": "UNKNOWN:0003",
  "gene_symbol": "ABTB3",
  "gene": "UniProtKB:A6QL63",
  "gene_name": "Ankyrin repeat and BTB_POZ domain-containing protein 3"
}